symbiont-mediated suppression of host T-cell mediated immune response [GO:0052085] (biological process) Also known as: negative regulation by organism of T-cell mediated immune response of other organism involved in symbiotic interaction, down regulation by symbiont of host T-cell mediated immune response, down-regulation by symbiont of host T-cell mediated immune response, downregulation by symbiont of host T-cell mediated immune response, negative regulation by symbiont of host T-cell mediated immune response, suppression by symbiont of host T-cell mediated immune response, suppression of host T-cell mediated immune response, inhibition by symbiont of host T-cell mediated immune response Sources: GOC:mtg_pamgo_17jul06 Definition: A process by which a symbiont interferes with, inhibits or disrupts the normal execution of the T-cell mediated immune response of the host organism. The host is defined as the larger of the organisms involved in a symbiotic interaction. Relationships: is a type of symbiont-mediated suppression of host adaptive immune response [GO:0039504]; is a type of symbiont-mediated perturbation of host T-cell mediated immune response [GO:0052156]